{
  "gene_name": "Nectin-3",
  "term_label": "cell adhesion mediator activity",
  "gene_symbol": "NECTIN3",
  "term_id": "GO:0098631",
  "gene": "UniProtKB:Q9NQS3"
}